{
  "term_label": "extracellular space",
  "gene": "UniProtKB:Q96BQ1",
  "gene_name": "Protein FAM3D",
  "gene_symbol": "FAM3D",
  "term_id": "GO:0005615"
}